{
  "gene_symbol": "C19orf73",
  "term_id": "UNKNOWN:0002",
  "term_label": "Unknown biological process",
  "gene_name": "Putative uncharacterized protein C19orf73",
  "gene": "UniProtKB:Q9NVV2"
}